{
  "gene": "UniProtKB:Q9NP55",
  "gene_symbol": "BPIFA1",
  "term_id": "UNKNOWN:0001",
  "gene_name": "BPI fold-containing family A member 1",
  "term_label": "Unknown molecular function"
}